{
  "gene": "UniProtKB:Q9BV99",
  "gene_symbol": "LRRC61",
  "term_label": "Unknown molecular function",
  "gene_name": "Leucine-rich repeat-containing protein 61",
  "term_id": "UNKNOWN:0001"
}